cellular bud neck [GO:0005935] (cellular component) Relationships: is a type of site of polarized growth [GO:0030427]; is part of cellular bud [GO:0005933] Sources: GOC:mah Definition: The constriction between the mother cell and daughter cell (bud) in an organism that reproduces by budding.